regulation of ventricular cardiac muscle cell action potential [GO:0098911] (biological process) Definition: Any process that modulates the frequency, rate or extent of action potential creation, propagation or termination in a ventricular cardiac muscle cell contributing to the regulation of its contraction. This typically occurs via modulation of the activity or expression of voltage-gated ion channels. Sources: GOC:BHF, GOC:mtg_cardiac_conduct_nov11 Relationships: is a type of regulation of cardiac muscle cell contraction [GO:0086004]; is a type of regulation of cardiac muscle cell action potential [GO:0098901]; regulates ventricular cardiac muscle cell action potential [GO:0086005] Subtypes: negative regulation of ventricular cardiac muscle cell action potential [GO:1903946], positive regulation of ventricular cardiac muscle cell action potential [GO:1903947]